retinol metabolic process [GO:0042572] (biological process) References: PMID:1924551 Sources: GOC:jl Relationships: is a type of GO:0001523; is a type of primary alcohol metabolic process [GO:0034308]; is a type of GO:0042445; is a type of olefinic compound metabolic process [GO:0120254] Also known as: retinol metabolism, vitamin A1 alcohol metabolic process, vitamin A1 alcohol metabolism, vitamin A1 metabolic process, vitamin A1 metabolism Definition: The chemical reactions and pathways involving retinol, one of the three compounds that makes up vitamin A.